{
  "term_id": "GO:0015175",
  "gene_symbol": "SLC1A2",
  "gene": "UniProtKB:P43004",
  "term_label": "neutral L-amino acid transmembrane transporter activity",
  "gene_name": "Excitatory amino acid transporter 2"
}